{
  "gene_name": "E3 ubiquitin-protein ligase TRIM39",
  "gene": "UniProtKB:Q9HCM9",
  "gene_symbol": "TRIM39",
  "term_label": "cytoplasm",
  "term_id": "GO:0005737"
}